{
  "term_label": "positive regulation of immune response",
  "gene_symbol": "HLA-DQB1",
  "gene_name": "HLA class II histocompatibility antigen, DQ beta 1 chain",
  "gene": "UniProtKB:P01920",
  "term_id": "GO:0050778"
}